leucine-tRNA ligase activity [GO:0004823] (molecular function) Definition: Catalysis of the reaction: leucine + ATP + tRNA(Leu) = AMP + diphosphate + 2 H+ + Leu-tRNA(Leu). Sources: RHEA:11688 Also known as: leucyl-tRNA synthetase activity, leucine translase activity, leucine-tRNA synthetase activity, leucine:tRNALeu ligase (AMP-forming), leucyl-transfer RNA synthetase activity, leucyl-transfer ribonucleate synthetase activity, leucyl-transfer ribonucleic acid synthetase activity Relationships: is a type of GO:0004812